motilin receptor binding [GO:0031788] (molecular function) Also known as: motilin receptor ligand Definition: Binding to a motilin receptor. Sources: GOC:mah, GOC:nln Relationships: is a type of G protein-coupled receptor binding [GO:0001664]